{
  "gene": "UniProtKB:Q7RTS7",
  "gene_symbol": "KRT74",
  "term_label": "intermediate filament organization",
  "term_id": "GO:0045109",
  "gene_name": "Keratin, type II cytoskeletal 74"
}